{
  "term_id": "GO:0030674",
  "term_label": "protein-macromolecule adaptor activity",
  "gene_name": "SH3 domain-containing protein 21",
  "gene": "UniProtKB:A4FU49",
  "gene_symbol": "SH3D21"
}